{
  "gene": "UniProtKB:P58872",
  "term_label": "Unknown cellular component",
  "gene_name": "Rhomboid-related protein 3",
  "term_id": "UNKNOWN:0003",
  "gene_symbol": "RHBDL3"
}